Kv4.1-DPP10 channel complex [GO:0071199] (cellular component) Definition: A voltage-gated potassium channel complex that contains the peptidase-related protein DPP10 associated with the channel via interaction with the Kv alpha subunit 4.1. References: PMID:15911355 Also known as: Kv4.1-DPPY channel complex Relationships: is a type of voltage-gated potassium channel complex [GO:0008076]